{
  "gene_symbol": "HINFP",
  "term_id": "GO:0006357",
  "gene_name": "Histone H4 transcription factor",
  "term_label": "regulation of transcription by RNA polymerase II",
  "gene": "UniProtKB:Q9BQA5"
}